{
  "term_id": "UNKNOWN:0002",
  "gene_symbol": "OR4D6",
  "gene_name": "Olfactory receptor 4D6",
  "term_label": "Unknown biological process",
  "gene": "UniProtKB:Q8NGJ1"
}